{
  "gene": "UniProtKB:P61018",
  "gene_symbol": "RAB4B",
  "term_label": "recycling endosome",
  "gene_name": "Ras-related protein Rab-4B",
  "term_id": "GO:0055037"
}